peripheral nervous system neuron differentiation [GO:0048934] (biological process) Sources: GOC:dgh Relationships: is a type of neuron differentiation [GO:0030182]; is part of peripheral nervous system development [GO:0007422] Definition: The process in which a relatively unspecialized cell acquires specialized features of a neuron whose cell body resides in the peripheral nervous system. Subtypes: lateral line ganglion neuron differentiation [GO:0048891], cardiac neuron differentiation [GO:0060945]